{
  "gene": "UniProtKB:Q93038",
  "term_id": "UNKNOWN:0001",
  "term_label": "Unknown molecular function",
  "gene_symbol": "TNFRSF25",
  "gene_name": "Tumor necrosis factor receptor superfamily member 25"
}